lens fiber cell differentiation [GO:0070306] (biological process) Also known as: lens fibre cell differentiation Definition: The process in which a relatively unspecialized cell acquires specialized features of a lens fiber cell, any of the elongated, tightly packed cells that make up the bulk of the mature lens in the camera-type eye. The cytoplasm of a lens fiber cell is devoid of most intracellular organelles including the cell nucleus, and contains primarily crystallins, a group of water-soluble proteins expressed in vary large quantities. Regulation: regulated by regulation of lens fiber cell differentiation [GO:1902746]; negatively regulated by negative regulation of lens fiber cell differentiation [GO:1902747]; positively regulated by positive regulation of lens fiber cell differentiation [GO:1902748] Relationships: is_a GO:0030855; is part of GO:0002088 References: PMID:7693735 Sources: GOC:mah